{
  "term_label": "RNA polymerase II core promoter sequence-specific DNA binding",
  "gene_name": "Transcription initiation factor IIB",
  "term_id": "GO:0000979",
  "gene": "UniProtKB:Q00403",
  "gene_symbol": "GTF2B"
}